small molecule biosynthetic process [GO:0044283] (BP) Also known as: small molecule biosynthesis Note: Small molecules in GO include monosaccharides but exclude disaccharides and polysaccharides. Relationships: is a type of GO:0009058; is a type of GO:0044281 Subtypes: hypochlorous acid biosynthetic process [GO:0002149], GO:0009110, organic acid biosynthetic process [GO:0016053], nucleobase-containing small molecule biosynthetic process [GO:0034404], urate biosynthetic process [GO:0034418], ketone biosynthetic process [GO:0042181], alcohol biosynthetic process [GO:0046165], GO:0046293, GO:0046364, ketone body biosynthetic process [GO:0046951] Sources: GOC:curators, GOC:pde, GOC:vw Definition: The chemical reactions and pathways resulting in the formation of small molecules, any low molecular weight, monomeric, non-encoded molecule.